detection of hypoxic conditions in blood by carotid body chemoreceptor signaling [GO:0003029] (biological process) Also known as: detection of hypoxic conditions in blood by carotid body chemoreceptor signalling Definition: The process in which information about a lack of oxygen are received and are converted to a molecular signal by chemoreceptors in the carotid bodies. Sources: GOC:mtg_cardio Relationships: is a type of GO:0002007; is part of regulation of systemic arterial blood pressure by carotid body chemoreceptor signaling [GO:0003027]